{
  "gene_symbol": "RILPL1",
  "gene_name": "RILP-like protein 1",
  "term_label": "cilium assembly",
  "term_id": "GO:0060271",
  "gene": "UniProtKB:Q5EBL4"
}